{
  "term_label": "Unknown biological process",
  "gene_name": "Cell division control protein 24 OB domain-containing protein",
  "term_id": "UNKNOWN:0002",
  "gene_symbol": "MGC35212",
  "gene": "UniProtKB:H3BU10"
}